{
  "term_id": "GO:1990414",
  "gene": "UniProtKB:Q6KC79",
  "gene_name": "Nipped-B-like protein",
  "gene_symbol": "NIPBL",
  "term_label": "replication-born double-strand break repair via sister chromatid exchange"
}